{
  "term_label": "Unknown biological process",
  "gene_name": "Putative uncharacterized protein FLJ42102",
  "term_id": "UNKNOWN:0002",
  "gene": "UniProtKB:Q6ZVU0",
  "gene_symbol": "Q6ZVU0"
}